nucleobase-containing compound metabolic process [GO:0006139] (biological process) Relationships: is a type of primary metabolic process [GO:0044238] Subtypes: nucleobase-containing compound biosynthetic process [GO:0034654], nucleobase-containing compound catabolic process [GO:0034655], nucleobase-containing small molecule metabolic process [GO:0055086], nucleic acid metabolic process [GO:0090304], polynucleotide 3' dephosphorylation [GO:0098506], polynucleotide 5' dephosphorylation [GO:0098507] Regulation: regulated by regulation of nucleobase-containing compound metabolic process [GO:0019219]; negatively regulated by negative regulation of nucleobase-containing compound metabolic process [GO:0045934] Definition: Any cellular metabolic process involving nucleobases, nucleosides, nucleotides and nucleic acids. Also known as: cellular nucleobase, nucleoside, nucleotide and nucleic acid metabolic process, cellular nucleobase, nucleoside, nucleotide and nucleic acid metabolism, nucleobase, nucleoside, nucleotide and nucleic acid metabolism, nucleobase, nucleoside and nucleotide metabolic process, nucleobase, nucleoside, nucleotide and nucleic acid metabolic process Sources: GOC:ai